{
  "term_label": "fibroblast growth factor receptor binding",
  "gene_name": "Fibroblast growth factor 4",
  "term_id": "GO:0005104",
  "gene_symbol": "FGF4",
  "gene": "UniProtKB:P08620"
}